{
  "term_label": "carbohydrate catabolic process",
  "gene_symbol": "DERA",
  "gene": "UniProtKB:Q9Y315",
  "term_id": "GO:0016052",
  "gene_name": "Deoxyribose-phosphate aldolase"
}